odontogenesis [GO:0042476] (biological process) Regulation: regulated by regulation of odontogenesis [GO:0042481]; positively regulated by GO:0042482; negatively regulated by negative regulation of odontogenesis [GO:0042483] Subtypes: odontogenesis of dentin-containing tooth [GO:0042475], tooth replacement [GO:0061648] Relationships: is a type of animal organ morphogenesis [GO:0009887] Also known as: odontogeny, odontosis, tooth morphogenesis, odontogenesis of calcareous or chitinous tooth, tooth development Definition: The process whose specific outcome is the progression of a tooth or teeth over time, from formation to the mature structure(s). A tooth is any hard bony, calcareous, or chitinous organ found in the mouth or pharynx of an animal and used in procuring or masticating food. Sources: GOC:jl, GOC:mah